{
  "term_id": "GO:0004477",
  "gene": "UniProtKB:P11586",
  "gene_name": "C-1-tetrahydrofolate synthase, cytoplasmic",
  "term_label": "methenyltetrahydrofolate cyclohydrolase activity",
  "gene_symbol": "MTHFD1"
}